{
  "term_label": "translation repressor activity",
  "gene_symbol": "EIF4EBP2",
  "gene_name": "Eukaryotic translation initiation factor 4E-binding protein 2",
  "term_id": "GO:0030371",
  "gene": "UniProtKB:Q13542"
}